positive regulation of adaptive immune effector response [GO:1905679] (biological process) Also known as: up regulation of adaptive immune effector response, up-regulation of adaptive immune effector response, upregulation of adaptive immune effector response, activation of adaptive immune effector response Sources: GOC:TermGenie, GO_REF:0000058, ISBN:9781405196833 Relationships: is a type of positive regulation of adaptive immune response [GO:0002821]; is a type of regulation of adaptive immune effector response [GO:1905677]; positively regulates GO:0090718 Definition: Any process that activates or increases the frequency, rate or extent of adaptive immune effector response.